{
  "gene_name": "Transducin-like enhancer protein 2",
  "gene": "UniProtKB:Q04725",
  "term_id": "GO:0090090",
  "term_label": "negative regulation of canonical Wnt signaling pathway",
  "gene_symbol": "TLE2"
}